cellular response to 2-O-acetyl-1-O-hexadecyl-sn-glycero-3-phosphocholine [GO:1904317] (BP) Definition: Any process that results in a change in state or activity of a cell (in terms of movement, secretion, enzyme production, gene expression, etc.) as a result of a 2-O-acetyl-1-O-hexadecyl-sn-glycero-3-phosphocholine stimulus. References: PMID:9321918 Sources: GOC:TermGenie, GO_REF:0000071 Also known as: cellular response to PAF, cellular response to platelet-activating factor Relationships: is_a cellular response to ether [GO:0071362]; is a type of cellular response to lipid [GO:0071396]; is a type of cellular response to nitrogen compound [GO:1901699]; is a type of response to 2-O-acetyl-1-O-hexadecyl-sn-glycero-3-phosphocholine [GO:1904316]